{
  "gene": "UniProtKB:Q8N137",
  "gene_symbol": "CNTROB",
  "gene_name": "Centrobin",
  "term_id": "GO:1902410",
  "term_label": "mitotic cytokinetic process"
}